{
  "term_id": "GO:0035189",
  "gene_symbol": "RB1",
  "gene": "UniProtKB:P06400",
  "term_label": "Rb-E2F complex",
  "gene_name": "Retinoblastoma-associated protein"
}